{
  "term_id": "UNKNOWN:0003",
  "gene": "UniProtKB:Q02505",
  "gene_name": "Mucin-3A",
  "term_label": "Unknown cellular component",
  "gene_symbol": "MUC3A"
}